response to topoisomerase inhibitor [GO:0072758] (biological process) Relationships: is a type of response to chemical [GO:0042221] Sources: GOC:mah Definition: Any process that results in a change in state or activity of a cell or an organism (in terms of movement, secretion, enzyme production, gene expression, etc.) as a result of a topoisomerase inhibitor stimulus. Subtypes: cellular response to topoisomerase inhibitor [GO:0072759]